{
  "term_label": "plasma membrane",
  "term_id": "GO:0005886",
  "gene": "UniProtKB:Q12955",
  "gene_name": "Ankyrin-3",
  "gene_symbol": "ANK3"
}